{
  "term_id": "GO:0031647",
  "term_label": "regulation of protein stability",
  "gene": "UniProtKB:Q9NVE5",
  "gene_symbol": "USP40",
  "gene_name": "Ubiquitin carboxyl-terminal hydrolase 40"
}